{
  "gene": "UniProtKB:Q96LR2",
  "gene_symbol": "LURAP1",
  "term_id": "UNKNOWN:0001",
  "term_label": "Unknown molecular function",
  "gene_name": "Leucine rich adaptor protein 1"
}